{
  "term_id": "GO:0000981",
  "term_label": "DNA-binding transcription factor activity, RNA polymerase II-specific",
  "gene_symbol": "ZNF433",
  "gene": "UniProtKB:Q8N7K0",
  "gene_name": "Zinc finger protein 433"
}